{
  "gene": "UniProtKB:A2CJ06",
  "term_label": "plasma membrane",
  "gene_name": "Dystrotelin",
  "gene_symbol": "DYTN",
  "term_id": "GO:0005886"
}